{
  "gene_symbol": "CCNT1",
  "gene": "UniProtKB:O60563",
  "gene_name": "Cyclin-T1",
  "term_label": "cyclin-dependent protein serine/threonine kinase activator activity",
  "term_id": "GO:0061575"
}